{
  "gene_symbol": "LIG4",
  "term_label": "DNA binding",
  "gene_name": "DNA ligase 4",
  "term_id": "GO:0003677",
  "gene": "UniProtKB:P49917"
}